{
  "gene_name": "Endogenous retroviral envelope protein HEMO",
  "gene": "UniProtKB:Q9H9K5",
  "term_id": "UNKNOWN:0001",
  "gene_symbol": "ERVMER34-1",
  "term_label": "Unknown molecular function"
}